{
  "gene_name": "tRNA pseudouridine synthase-like 1",
  "gene": "UniProtKB:Q8N0Z8",
  "term_id": "GO:0009982",
  "gene_symbol": "PUSL1",
  "term_label": "pseudouridine synthase activity"
}